{
  "gene_symbol": "ZNF419",
  "gene": "UniProtKB:Q96HQ0",
  "term_id": "GO:0005634",
  "term_label": "nucleus",
  "gene_name": "Zinc finger protein 419"
}